{
  "gene_name": "ATP-dependent RNA helicase A",
  "term_id": "GO:0005730",
  "gene": "UniProtKB:Q08211",
  "term_label": "nucleolus",
  "gene_symbol": "DHX9"
}